{
  "term_label": "synaptic vesicle docking",
  "term_id": "GO:0016081",
  "gene_symbol": "RIMS3",
  "gene": "UniProtKB:Q9UJD0",
  "gene_name": "Regulating synaptic membrane exocytosis protein 3"
}